{
  "gene": "UniProtKB:P78396",
  "term_id": "GO:0097124",
  "gene_symbol": "CCNA1",
  "gene_name": "Cyclin-A1",
  "term_label": "cyclin A2-CDK2 complex"
}